dermatan sulfotransferase activity [GO:0120534] (molecular function) Subtypes: GO:0001537, dermatan 2-sulfotransferase activity [GO:0102142] Relationships: is a type of proteoglycan sulfotransferase activity [GO:0050698] Definition: Catalysis of the reaction: 3'-phosphoadenylyl sulfate + dermatan = adenosine 3',5'-bisphosphate + dermatan sulfate. Sources: GOC:curators